{
  "term_id": "GO:0015810",
  "gene": "UniProtKB:Q8IWT6",
  "term_label": "aspartate transmembrane transport",
  "gene_symbol": "LRRC8A",
  "gene_name": "Volume-regulated anion channel subunit LRRC8A"
}